{
  "gene": "UniProtKB:Q9NQG6",
  "gene_name": "Mitochondrial dynamics protein MIEF1",
  "gene_symbol": "MIEF1",
  "term_id": "GO:0005741",
  "term_label": "mitochondrial outer membrane"
}